{
  "gene_symbol": "H3-5",
  "term_label": "kinetochore",
  "gene_name": "Histone H3.3C",
  "term_id": "GO:0000776",
  "gene": "UniProtKB:Q6NXT2"
}